{
  "gene_symbol": "MSTO1",
  "gene_name": "Protein misato homolog 1",
  "gene": "UniProtKB:Q9BUK6",
  "term_id": "UNKNOWN:0001",
  "term_label": "Unknown molecular function"
}